{
  "term_label": "plasma membrane",
  "term_id": "GO:0005886",
  "gene": "UniProtKB:A0A075B6N2",
  "gene_name": "T cell receptor beta variable 20-1",
  "gene_symbol": "TRBV20-1"
}